{
  "gene": "UniProtKB:Q9BX68",
  "gene_name": "Adenosine 5'-monophosphoramidase HINT2",
  "term_label": "cytoplasm",
  "gene_symbol": "HINT2",
  "term_id": "GO:0005737"
}